rhabdomere microvillus [GO:0035996] (cellular component) Relationships: is a type of microvillus [GO:0005902]; is part of rhabdomere [GO:0016028] References: PMID:14744998 Sources: GOC:bf, GOC:sart Definition: Thin cylindrical membrane-covered projection on the surface of a rhabdomere.